{
  "term_id": "GO:0035556",
  "gene_symbol": "PRKD1",
  "gene": "UniProtKB:Q15139",
  "term_label": "intracellular signal transduction",
  "gene_name": "Serine_threonine-protein kinase D1"
}